{
  "term_id": "UNKNOWN:0003",
  "term_label": "Unknown cellular component",
  "gene_symbol": "TNFRSF8",
  "gene": "UniProtKB:P28908",
  "gene_name": "Tumor necrosis factor receptor superfamily member 8"
}